{
  "gene": "UniProtKB:Q9NRR6",
  "term_id": "GO:0046856",
  "gene_symbol": "INPP5E",
  "term_label": "phosphatidylinositol dephosphorylation",
  "gene_name": "Phosphatidylinositol polyphosphate 5-phosphatase type IV"
}